{
  "gene_name": "Membrane protein FAM174A",
  "term_id": "UNKNOWN:0003",
  "gene_symbol": "FAM174A",
  "term_label": "Unknown cellular component",
  "gene": "UniProtKB:Q8TBP5"
}